proctolin receptor binding [GO:0071860] (molecular function) Definition: Binding to a proctolin receptor. Relationships: is a type of neuropeptide receptor binding [GO:0071855] Sources: GOC:kmv, GOC:mah